{
  "gene": "UniProtKB:Q6P3X3",
  "gene_symbol": "TTC27",
  "gene_name": "Tetratricopeptide repeat protein 27",
  "term_id": "UNKNOWN:0002",
  "term_label": "Unknown biological process"
}